RNA polymerase I core binding [GO:0001042] (molecular function) Relationships: is a type of GO:0043175 Definition: Binding to a RNA polymerase I core enzyme, a multisubunit eukaryotic nuclear RNA polymerase typically composed of seventeen subunits. Sources: GOC:txnOH